{
  "gene": "UniProtKB:O14730",
  "term_id": "GO:0030688",
  "gene_name": "Serine_threonine-protein kinase RIO3",
  "term_label": "preribosome, small subunit precursor",
  "gene_symbol": "RIOK3"
}